4-(cytidine 5'-diphospho)-2-C-methyl-D-erythritol kinase activity [GO:0050515] (molecular function) Sources: EC:2.7.1.148, RHEA:18437 Also known as: 4-diphosphocytidyl-2C-methyl-D-erythritol kinase activity, 4-diphosphocytidyl-2-C-methyl-D-erythritol kinase activity, ATP:4-(cytidine 5'-diphospho)-2-C-methyl-D-erythritol 2-phosphotransferase activity, CDP-ME kinase activity, CMK activity Relationships: is a type of kinase activity [GO:0016301]; is a type of phosphotransferase activity, alcohol group as acceptor [GO:0016773] Definition: Catalysis of the reaction: 4-CDP-2-C-methyl-D-erythritol + ATP = 4-CDP-2-C-methyl-D-erythritol 2-phosphate + ADP + 2 H+.